gentisate 1,2-dioxygenase activity [GO:0047922] (molecular function) Sources: EC:1.13.11.4, RHEA:18237 Relationships: is_a GO:0016702 Also known as: 2,5-dihydroxybenzoate dioxygenase activity, gentisate dioxygenase activity, gentisate oxygenase activity, gentisate:oxygen 1,2-oxidoreductase (decyclizing), gentisic acid oxidase activity Definition: Catalysis of the reaction: 2,5-dihydroxybenzoate + O2 = 3-maleylpyruvate + H+.